{
  "term_id": "GO:0005886",
  "term_label": "plasma membrane",
  "gene_name": "Uncharacterized protein KIAA1755",
  "gene": "UniProtKB:Q5JYT7",
  "gene_symbol": "KIAA1755"
}